{
  "term_label": "GTPase activator activity",
  "term_id": "GO:0005096",
  "gene": "UniProtKB:O14921",
  "gene_name": "Regulator of G-protein signaling 13",
  "gene_symbol": "RGS13"
}